{
  "term_id": "GO:2000330",
  "term_label": "positive regulation of T-helper 17 cell lineage commitment",
  "gene": "UniProtKB:Q9NPF7",
  "gene_name": "Interleukin-23 subunit alpha",
  "gene_symbol": "IL23A"
}